negative regulation of cell fate specification [GO:0009996] (biological process) Definition: Any process that restricts, stops or prevents a cell from adopting a specific cell fate. Sources: GOC:go_curators Relationships: is a type of negative regulation of cell fate commitment [GO:0010454]; is a type of GO:0042659; negatively regulates cell fate specification [GO:0001708] Also known as: down regulation of cell fate specification, down-regulation of cell fate specification, downregulation of cell fate specification, suppression of cell fate, inhibition of cell fate specification Subtypes: negative regulation of retinal cone cell fate specification [GO:0009998], negative regulation of auditory receptor cell fate specification [GO:0009999], negative regulation of atrichoblast fate specification [GO:0010060], negative regulation of trichoblast fate specification [GO:0010062], negative regulation of terminal cell fate specification, open tracheal system [GO:0035155], GO:0035157, negative regulation of mesodermal cell fate specification [GO:0042662], negative regulation of endodermal cell fate specification [GO:0042664], negative regulation of ectodermal cell fate specification [GO:0042666], GO:0042683, negative regulation of neural crest cell fate specification [GO:1905296], GO:2000044